{
  "gene": "UniProtKB:Q53H64",
  "gene_name": "Putative ANKRD40 C-terminal-like protein",
  "term_label": "Unknown biological process",
  "gene_symbol": "ANKRD40CL",
  "term_id": "UNKNOWN:0002"
}